{
  "gene_symbol": "USP50",
  "gene_name": "Inactive ubiquitin carboxyl-terminal hydrolase 50",
  "term_label": "cysteine-type deubiquitinase activity",
  "term_id": "GO:0004843",
  "gene": "UniProtKB:Q70EL3"
}